jasmonic acid mediated signaling pathway [GO:0009867] (biological process) Relationships: is a type of GO:0009755; is part of GO:0071395 Regulation: regulated by regulation of jasmonic acid mediated signaling pathway [GO:2000022] References: PMID:16478936, PMID:19522558, PMID:20159850 Sources: GOC:jy Also known as: JA signaling, jasmonic acid mediated signalling pathway, jasmonate signaling Subtypes: induced systemic resistance, jasmonic acid mediated signaling pathway [GO:0009864], jasmonic acid and ethylene-dependent systemic resistance, jasmonic acid mediated signaling pathway [GO:0009868] Definition: The series of molecular signals mediated by jasmonic acid.